{
  "gene_symbol": "OSBPL7",
  "term_id": "GO:0031965",
  "gene_name": "Oxysterol-binding protein-related protein 7",
  "term_label": "nuclear membrane",
  "gene": "UniProtKB:Q9BZF2"
}